{
  "gene": "UniProtKB:O43516",
  "term_label": "actin filament",
  "gene_symbol": "WIPF1",
  "term_id": "GO:0005884",
  "gene_name": "WAS_WASL-interacting protein family member 1"
}